sphingomyelin phosphodiesterase activity [GO:0004767] (molecular function) Relationships: is a type of GO:0004620; is_a GO:0008081 Also known as: sphingomyelinase activity, sphingomyelin cholinephosphohydrolase activity Subtypes: acid sphingomyelin phosphodiesterase activity [GO:0061750], neutral sphingomyelin phosphodiesterase activity [GO:0061751] Regulation: positively regulated by sphingomyelin phosphodiesterase activator activity [GO:0016230] Definition: Catalysis of the reaction: H2O + sphingomyelin = ceramide + choline phosphate + H+. Sources: EC:3.1.4.12, RHEA:19253